{
  "term_label": "semaphorin-plexin signaling pathway",
  "gene": "UniProtKB:Q8NFY4",
  "gene_name": "Semaphorin-6D",
  "term_id": "GO:0071526",
  "gene_symbol": "SEMA6D"
}